specification of plant organ number [GO:0048832] (BP) Sources: GOC:dph, GOC:isa_complete, GOC:tb Subtypes: specification of floral organ number [GO:0048833] Definition: The regionalization process that modulates the quantity of a particular type of plant organ. Relationships: is a type of regionalization [GO:0003002]; is a type of regulation of developmental process [GO:0050793]